esculin beta-glucosidase activity [GO:0080082] (molecular function) Definition: Catalysis of the hydrolysis of glucosidic link in esculin. References: PMID:15604686 Relationships: is a type of beta-glucosidase activity [GO:0008422]